cardiac chamber ballooning [GO:0003242] (biological process) Definition: The morphogenic growth in which the chambers of the heart expand in size, contributing to their shaping. Relationships: is a type of growth involved in heart morphogenesis [GO:0003241]; is part of cardiac chamber morphogenesis [GO:0003206] Sources: GOC:mtg_heart